multivesicular body, internal vesicle membrane [GO:0097488] (cellular component) Definition: The lipid bilayer surrounding a multivesicular body internal vesicle. References: PMID:21183070 Sources: GOC:pde Relationships: is a type of cytoplasmic vesicle membrane [GO:0030659]; is a type of bounding membrane of organelle [GO:0098588]; is part of GO:0097487